positive regulation of response to acetate [GO:1901459] (biological process) Sources: GOC:TermGenie, GOC:mengo_curators Also known as: up regulation of response to acetate, up-regulation of response to acetate, upregulation of response to acetate, activation of response to acetate Definition: Any process that activates or increases the frequency, rate or extent of response to acetate. Relationships: is_a positive regulation of response to stimulus [GO:0048584]; is a type of regulation of response to acetate [GO:1901457]; positively regulates response to acetate [GO:0010034]